{
  "gene_name": "Aspartyl_asparaginyl beta-hydroxylase",
  "gene_symbol": "ASPH",
  "term_label": "endoplasmic reticulum",
  "term_id": "GO:0005783",
  "gene": "UniProtKB:Q12797"
}